{
  "gene_symbol": "TAF11L5",
  "gene": "UniProtKB:A0A1W2PP81",
  "term_label": "transcription factor TFIID complex",
  "gene_name": "TATA-box-binding protein-associated factor 11-like protein 5",
  "term_id": "GO:0005669"
}